{
  "term_id": "GO:0006508",
  "gene_name": "Calpain-7",
  "gene_symbol": "CAPN7",
  "term_label": "proteolysis",
  "gene": "UniProtKB:Q9Y6W3"
}